{
  "term_id": "UNKNOWN:0001",
  "gene": "UniProtKB:Q96HR9",
  "gene_name": "Receptor expression-enhancing protein 6",
  "gene_symbol": "REEP6",
  "term_label": "Unknown molecular function"
}